{
  "gene_symbol": "H3-3B",
  "gene": "UniProtKB:P84243",
  "term_id": "GO:0007080",
  "term_label": "mitotic metaphase chromosome alignment",
  "gene_name": "Histone H3.3"
}